metal incorporation into metallo-molybdopterin complex [GO:0042040] (biological process) Relationships: is a type of protein modification process [GO:0036211] Subtypes: molybdenum incorporation into molybdenum-molybdopterin complex [GO:0018315], tungsten incorporation into tungsten-molybdopterin complex [GO:0042042] Sources: GOC:ai Definition: The incorporation of a metal into a metallo-molybdopterin complex.